{
  "term_label": "membrane",
  "term_id": "GO:0016020",
  "gene_name": "UPF0764 protein C16orf89",
  "gene": "UniProtKB:Q6UX73",
  "gene_symbol": "C16orf89"
}